{
  "gene_symbol": "CALCB",
  "gene": "UniProtKB:P10092",
  "term_id": "GO:0051480",
  "gene_name": "Calcitonin gene-related peptide 2",
  "term_label": "regulation of cytosolic calcium ion concentration"
}